{
  "gene_symbol": "FAM161B",
  "term_label": "Unknown cellular component",
  "term_id": "UNKNOWN:0003",
  "gene_name": "Protein FAM161B",
  "gene": "UniProtKB:Q96MY7"
}